{
  "gene": "UniProtKB:P05556",
  "gene_symbol": "ITGB1",
  "term_id": "GO:0005178",
  "term_label": "integrin binding",
  "gene_name": "Integrin beta-1"
}